{
  "gene": "UniProtKB:Q8TF21",
  "gene_name": "Ankyrin repeat domain-containing protein 24",
  "term_id": "UNKNOWN:0003",
  "gene_symbol": "ANKRD24",
  "term_label": "Unknown cellular component"
}